regulation of CD4-positive, CD25-positive, alpha-beta regulatory T cell differentiation [GO:0032829] (biological process) Also known as: regulation of CD4-positive, CD25-positive, alpha-beta regulatory T lymphocyte differentiation, regulation of CD4-positive, CD25-positive, alpha-beta regulatory T-cell differentiation, regulation of CD4-positive, CD25-positive, alpha-beta regulatory T-lymphocyte differentiation, regulation of CD4-positive, CD25-positive, alpha-beta regulatory T cell development Subtypes: negative regulation of CD4-positive, CD25-positive, alpha-beta regulatory T cell differentiation [GO:0032830], positive regulation of CD4-positive, CD25-positive, alpha-beta regulatory T cell differentiation [GO:0032831], GO:0032832 Note: Note that immunologists typically use the word 'development' to refer to cells of B or T cell lineages undergoing the process that GO describes as 'cell differentiation'. Relationships: is a type of regulation of CD4-positive, alpha-beta T cell differentiation [GO:0043370]; is a type of regulation of regulatory T cell differentiation [GO:0045589]; regulates GO:0002361 Definition: Any process that modulates the frequency, rate or extent of differentiation of CD4-positive, CD25-positive, alpha-beta regulatory T cells. Sources: GOC:mah